swarm social behavior [GO:0160306] (biological process) Definition: A social behavior in which multiple individuals of the same animal species coordinate their movement in close spatial proximity, forming a dynamic aggregation typically characterized by collective motion, cohesion, and mutual responsiveness among members of the group. Also known as: swarming behavior References: PMID:23740485, PMID:32788724 Sources: DOI:10.1007/s13592-013-0253-2 Relationships: is_a social behavior [GO:0035176]